pointed-end actin filament uncapping [GO:0051696] (biological process) Sources: GOC:pf Definition: The removal of capping protein from the pointed (or minus) end of actin filaments to free the ends for addition, exchange or removal of further actin subunits. Also known as: minus end F-actin uncapping, minus end actin filament uncapping, minus-end F-actin uncapping, minus-end actin filament uncapping, pointed end F-actin uncapping, pointed end actin filament uncapping, pointed-end F-actin uncapping Relationships: is a type of actin filament uncapping [GO:0051695]